{
  "term_id": "GO:0005737",
  "term_label": "cytoplasm",
  "gene_symbol": "PABIR1",
  "gene": "UniProtKB:Q96E09",
  "gene_name": "PPP2R1A-PPP2R2A-interacting phosphatase regulator 1"
}